{
  "gene_symbol": "ARRDC1-AS1",
  "term_label": "Unknown molecular function",
  "gene": "UniProtKB:Q9H2J1",
  "term_id": "UNKNOWN:0001",
  "gene_name": "Uncharacterized protein ARRDC1-AS1"
}